histidine ammonia-lyase activity [GO:0004397] (MF) Relationships: is a type of GO:0016841 Also known as: L-histidine ammonia-lyase (urocanate-forming), L-histidine ammonia-lyase activity, histidase activity, histidinase activity, histidine alpha-deaminase activity Definition: Catalysis of the reaction: L-histidine = urocanate + NH3. Sources: EC:4.3.1.3